{
  "gene": "UniProtKB:P08F94",
  "gene_name": "Fibrocystin",
  "term_id": "UNKNOWN:0003",
  "term_label": "Unknown cellular component",
  "gene_symbol": "PKHD1"
}